{
  "term_label": "cytoplasmic translation",
  "gene_name": "Large ribosomal subunit protein eL22",
  "gene_symbol": "RPL22",
  "gene": "UniProtKB:P35268",
  "term_id": "GO:0002181"
}